{
  "gene_name": "Polyubiquitin-B",
  "term_label": "nucleus",
  "gene": "UniProtKB:P0CG47",
  "term_id": "GO:0005634",
  "gene_symbol": "UBB"
}